{
  "term_label": "ubiquitin protein ligase binding",
  "gene": "UniProtKB:Q9BXW4",
  "gene_name": "Microtubule-associated proteins 1A_1B light chain 3C",
  "term_id": "GO:0031625",
  "gene_symbol": "MAP1LC3C"
}